{
  "gene_symbol": "CD207",
  "term_label": "immune response",
  "gene": "UniProtKB:Q9UJ71",
  "term_id": "GO:0006955",
  "gene_name": "C-type lectin domain family 4 member K"
}